negative regulation of interleukin-34 production [GO:0150159] (biological process) Also known as: negative regulation of interleukin-34 biosynthetic process References: PMID:26754294 Sources: GOC:aruk Relationships: is a type of negative regulation of cytokine production [GO:0001818]; is a type of GO:0150157; negatively regulates GO:0150155 Definition: Any process that stops, prevents or reduces the frequency, rate or extent of interleukin-34 production.